{
  "term_label": "cytoplasm",
  "gene": "UniProtKB:P54819",
  "gene_name": "Adenylate kinase 2, mitochondrial",
  "term_id": "GO:0005737",
  "gene_symbol": "AK2"
}